{
  "gene": "UniProtKB:P0DMU9",
  "term_label": "Unknown biological process",
  "gene_symbol": "CT45A10",
  "gene_name": "Cancer_testis antigen family 45 member A10",
  "term_id": "UNKNOWN:0002"
}